pre-mRNA catabolic process [GO:1990261] (biological process) Definition: The chemical reactions and pathways resulting in the breakdown of the unspliced pre-mRNA (pre-messenger RNA). References: PMID:22844259 Sources: GOC:rb Also known as: pre-mRNA decay, unspliced RNA decay Relationships: is a type of RNA catabolic process [GO:0006401]